{
  "gene": "UniProtKB:P78406",
  "term_id": "GO:0043130",
  "term_label": "ubiquitin binding",
  "gene_symbol": "RAE1",
  "gene_name": "mRNA export factor RAE1"
}